{
  "gene": "UniProtKB:Q9ULK5",
  "term_id": "GO:0005886",
  "gene_symbol": "VANGL2",
  "gene_name": "Vang-like protein 2",
  "term_label": "plasma membrane"
}